{
  "term_label": "Unknown biological process",
  "term_id": "UNKNOWN:0002",
  "gene_name": "Zinc finger HIT domain-containing protein 2",
  "gene": "UniProtKB:Q9UHR6",
  "gene_symbol": "ZNHIT2"
}